laminin-11 complex [GO:0043260] (cellular component) Definition: A laminin complex composed of alpha5, beta2 and gamma1 polypeptide chains. Relationships: is a type of laminin complex [GO:0043256] Also known as: laminin-521 complex References: PMID:10842354 Sources: GOC:jl